{
  "term_id": "GO:0008584",
  "gene": "UniProtKB:P22888",
  "term_label": "male gonad development",
  "gene_symbol": "LHCGR",
  "gene_name": "Lutropin-choriogonadotropic hormone receptor"
}